{
  "gene_symbol": "P2RY10",
  "gene_name": "Putative P2Y purinoceptor 10",
  "term_id": "GO:0007186",
  "gene": "UniProtKB:O00398",
  "term_label": "G protein-coupled receptor signaling pathway"
}